postsynaptic specialization membrane [GO:0099634] (cellular component) Definition: The membrane component of the postsynaptic specialization. This is the region of the postsynaptic membrane in which the population of neurotransmitter receptors involved in synaptic transmission are concentrated. Relationships: is a type of synaptic membrane [GO:0097060]; BFO_0000050 postsynaptic membrane [GO:0045211]; is part of postsynaptic specialization [GO:0099572] Sources: GOC:dos Subtypes: postsynaptic density membrane [GO:0098839], GO:0099164